{
  "gene": "UniProtKB:P20711",
  "gene_name": "Aromatic-L-amino-acid decarboxylase",
  "term_label": "cytoplasm",
  "term_id": "GO:0005737",
  "gene_symbol": "DDC"
}